{
  "gene": "UniProtKB:P51589",
  "term_label": "xenobiotic metabolic process",
  "gene_symbol": "CYP2J2",
  "term_id": "GO:0006805",
  "gene_name": "Cytochrome P450 2J2"
}